{
  "term_id": "GO:0005634",
  "gene_name": "26S proteasome non-ATPase regulatory subunit 2",
  "term_label": "nucleus",
  "gene_symbol": "PSMD2",
  "gene": "UniProtKB:Q13200"
}